flower structural organization [GO:0048461] (biological process) Definition: The process that contributes to the act of creating the structural organization of the flower. This process pertains to the physical shaping of a rudimentary structure. Sources: GOC:jid Also known as: flower structural organisation Relationships: is a type of developmental process involved in reproduction [GO:0003006]; is a type of GO:0048532; is part of GO:0048439